{
  "gene_symbol": "ZNF385A",
  "gene_name": "Zinc finger protein 385A",
  "term_id": "GO:0005634",
  "term_label": "nucleus",
  "gene": "UniProtKB:Q96PM9"
}